{
  "gene_symbol": "EID2B",
  "gene": "UniProtKB:Q96D98",
  "gene_name": "EP300-interacting inhibitor of differentiation 2B",
  "term_label": "negative regulation of DNA-templated transcription",
  "term_id": "GO:0045892"
}